{
  "term_label": "DNA-binding transcription factor activity, RNA polymerase II-specific",
  "gene_symbol": "GATAD2B",
  "term_id": "GO:0000981",
  "gene": "UniProtKB:Q8WXI9",
  "gene_name": "Transcriptional repressor p66-beta"
}